{
  "gene": "UniProtKB:Q76M96",
  "term_id": "GO:0030198",
  "gene_name": "Coiled-coil domain-containing protein 80",
  "term_label": "extracellular matrix organization",
  "gene_symbol": "CCDC80"
}